{
  "gene_symbol": "COMTD1",
  "term_label": "Unknown cellular component",
  "term_id": "UNKNOWN:0003",
  "gene": "UniProtKB:Q86VU5",
  "gene_name": "Catechol O-methyltransferase domain-containing protein 1"
}